{
  "term_id": "GO:0005509",
  "gene": "UniProtKB:Q96Q77",
  "gene_name": "Calcium and integrin-binding family member 3",
  "gene_symbol": "CIB3",
  "term_label": "calcium ion binding"
}